{
  "gene_symbol": "SPDYA",
  "term_id": "GO:0000082",
  "term_label": "G1/S transition of mitotic cell cycle",
  "gene_name": "Speedy protein A",
  "gene": "UniProtKB:Q5MJ70"
}